granulocyte-macrophage colony-stimulating factor signaling pathway [GO:0038157] (biological process) Also known as: CSF2 signaling pathway, GM-CSF receptor signaling pathway, GM-CSF signaling pathway, granulocyte-macrophage colony-stimulating factor receptor signaling pathway, granulocyte-macrophage colony-stimulating factor signalling pathway Relationships: is a type of cytokine-mediated signaling pathway [GO:0019221] Definition: The series of molecular signals initiated by the binding of the cytokine granulocyte macrophage colony-stimulating factor (GM-CSF) to its receptor on the surface of a target cell, and ending with the regulation of a downstream cellular process, e.g. transcription. GM-CSF binds to a heterodimer receptor (CSF2R) consisting of an alpha ligand-binding subunit, and a common beta subunit that is shared with other cytokine receptors. References: PMID:17027509 Sources: GOC:nhn, GOC:signaling